{
  "term_id": "GO:0005739",
  "gene": "UniProtKB:P05165",
  "gene_name": "Propionyl-CoA carboxylase alpha chain, mitochondrial",
  "gene_symbol": "PCCA",
  "term_label": "mitochondrion"
}